{
  "gene_name": "Interferon alpha-10",
  "gene_symbol": "IFNA10",
  "term_label": "B cell activation involved in immune response",
  "term_id": "GO:0002312",
  "gene": "UniProtKB:P01566"
}